{
  "term_label": "mitochondrion",
  "gene_symbol": "ALDH18A1",
  "gene_name": "Delta-1-pyrroline-5-carboxylate synthase",
  "gene": "UniProtKB:P54886",
  "term_id": "GO:0005739"
}